nucleobase-containing small molecule metabolic process [GO:0055086] (biological process) Definition: The cellular chemical reactions and pathways involving a nucleobase-containing small molecule: a nucleobase, a nucleoside, or a nucleotide. Also known as: nucleobase, nucleoside and nucleotide metabolism, nucleobase, nucleoside and nucleotide metabolic process Sources: GOC:vw Relationships: is a type of nucleobase-containing compound metabolic process [GO:0006139]; is a type of GO:0044281 Subtypes: GO:0006753, nucleobase metabolic process [GO:0009112], nucleoside metabolic process [GO:0009116], nucleobase-containing small molecule interconversion [GO:0015949], nucleobase-containing small molecule biosynthetic process [GO:0034404], nucleobase-containing small molecule catabolic process [GO:0034656]